{
  "gene": "UniProtKB:P08559",
  "term_label": "mitochondrion",
  "gene_symbol": "PDHA1",
  "gene_name": "Pyruvate dehydrogenase E1 component subunit alpha, somatic form, mitochondrial",
  "term_id": "GO:0005739"
}